cellular response to plumbagin [GO:1902709] (biological process) Relationships: is a type of GO:1901655; is a type of GO:1902708 Definition: Any process that results in a change in state or activity of a cell (in terms of movement, secretion, enzyme production, gene expression, etc.) as a result of a plumbagin stimulus. References: PMID:23028742 Sources: GOC:TermGenie, GO_REF:0000071